{
  "gene_name": "ALK tyrosine kinase receptor",
  "gene": "UniProtKB:Q9UM73",
  "gene_symbol": "ALK",
  "term_id": "GO:0043235",
  "term_label": "receptor complex"
}